regulation of B cell apoptotic process [GO:0002902] (biological process) Also known as: regulation of B cell apoptosis Sources: GOC:add, GOC:mtg_apoptosis Relationships: is a type of regulation of lymphocyte apoptotic process [GO:0070228]; regulates B cell apoptotic process [GO:0001783] Subtypes: regulation of B cell deletion [GO:0002867], negative regulation of B cell apoptotic process [GO:0002903], positive regulation of B cell apoptotic process [GO:0002904], regulation of mature B cell apoptotic process [GO:0002905] Definition: Any process that modulates the frequency, rate, or extent of B cell apoptotic process.